eosinophil extravasation [GO:0072682] (biological process) Definition: The migration of an eosinophil from the blood vessels into the surrounding tissue. Relationships: is a type of GO:0045123; is a type of GO:0072677 Regulation: regulated by regulation of eosinophil extravasation [GO:2000419]; negatively regulated by negative regulation of eosinophil extravasation [GO:2000420]; positively regulated by GO:2000421 Sources: CL:0000771, GOC:BHF, GOC:mah